interneuron migration from the subpallium to the cortex [GO:0021830] (biological process) Definition: The directed movement of interneurons from the subpallium to the cortex during forebrain development. References: PMID:12626695 Sources: GOC:cls, GOC:dgh, GOC:dph, GOC:jid, GO_REF:0000021 Relationships: is a type of substrate-independent telencephalic tangential interneuron migration [GO:0021843] Subtypes: cerebral cortex GABAergic interneuron migration [GO:0021853]